{
  "term_id": "UNKNOWN:0003",
  "gene_symbol": "ZSCAN31",
  "gene_name": "Zinc finger and SCAN domain-containing protein 31",
  "term_label": "Unknown cellular component",
  "gene": "UniProtKB:Q96LW9"
}